{
  "term_label": "Lsm1-7-Pat1 complex",
  "gene": "UniProtKB:P62310",
  "term_id": "GO:1990726",
  "gene_symbol": "LSM3",
  "gene_name": "U6 snRNA-associated Sm-like protein LSm3"
}